{
  "gene_symbol": "SERPINE1",
  "term_id": "GO:0061044",
  "gene": "UniProtKB:P05121",
  "term_label": "negative regulation of vascular wound healing",
  "gene_name": "Plasminogen activator inhibitor 1"
}